mRNA cap binding [GO:0098808] (molecular function) Relationships: is a type of RNA cap binding [GO:0000339]; is a type of GO:0003729 Sources: GOC:dos Definition: Binding to a 7-methylguanosine (m7G) group or derivative located at the 5' end of an mRNA molecule.